{
  "gene": "UniProtKB:P02818",
  "term_id": "GO:0046848",
  "term_label": "hydroxyapatite binding",
  "gene_symbol": "BGLAP",
  "gene_name": "Osteocalcin"
}